{
  "term_label": "negative regulation of viral genome replication",
  "gene_name": "Interferon-induced transmembrane protein 2",
  "gene_symbol": "IFITM2",
  "term_id": "GO:0045071",
  "gene": "UniProtKB:Q01629"
}